symbiont-mediated activation of host anti-inflammatory cytokine signaling [GO:0141184] (biological process) References: PMID:23284742, PMID:27437422, PMID:29924996 Definition: A process in which a symbiont subverts an anti-inflammatory cytokine signaling pathway in the host organism by initiating, promoting, or enhancing its activation. Relationships: is a type of GO:0052028